positive regulation of early endosome to recycling endosome transport [GO:1902955] (biological process) References: PMID:22621900 Sources: GOC:TermGenie, GOC:sjp, GO_REF:0000058 Also known as: up regulation of early endosome to recycling endosome transport, up-regulation of early endosome to recycling endosome transport, upregulation of early endosome to recycling endosome transport, activation of early endosome to recycling endosome transport Definition: Any process that activates or increases the frequency, rate or extent of early endosome to recycling endosome transport. Relationships: is a type of GO:0032388; is a type of regulation of early endosome to recycling endosome transport [GO:1902954]; positively regulates early endosome to recycling endosome transport [GO:0061502]